{
  "term_label": "cytoplasm",
  "term_id": "GO:0005737",
  "gene_name": "Serine_threonine-protein kinase ULK3",
  "gene": "UniProtKB:Q6PHR2",
  "gene_symbol": "ULK3"
}